{
  "term_id": "GO:0033490",
  "term_label": "cholesterol biosynthetic process via lathosterol",
  "gene_name": "Lathosterol oxidase",
  "gene_symbol": "SC5D",
  "gene": "UniProtKB:O75845"
}